{
  "gene_symbol": "SNRPN",
  "gene_name": "Small nuclear ribonucleoprotein-associated protein N",
  "term_id": "GO:0005685",
  "term_label": "U1 snRNP",
  "gene": "UniProtKB:P63162"
}